regulation of short-day photoperiodism, flowering [GO:0048587] (biological process) Relationships: is a type of GO:2000028; RO_0002211 short-day photoperiodism, flowering [GO:0048575] Definition: Any process that modulates the frequency, rate or extent of short-day photoperiodism, where the response associated with the photoperiodism is flowering. Flowering is defined by the switch from the vegetative to the reproductive phase. Subtypes: GO:0048576, GO:0048577 Sources: GOC:jid, GOC:pj, ISBN:0582015952, ISBN:0697037754, ISBN:0709408862